{
  "term_label": "Unknown biological process",
  "term_id": "UNKNOWN:0002",
  "gene_name": "Putative uncharacterized protein FLJ40288",
  "gene": "UniProtKB:A4D1N5",
  "gene_symbol": "A4D1N5"
}